amino acid activation for nonribosomal peptide biosynthetic process [GO:0043041] (biological process) Also known as: nonribosomal amino acid activation Sources: GOC:jl Subtypes: tRNA aminoacylation for nonribosomal peptide biosynthetic process [GO:0043040], amino acid adenylylation by nonribosomal peptide synthase [GO:0043042] Relationships: is a type of GO:0043038; is part of nonribosomal peptide biosynthetic process [GO:0019184] Definition: Activation of an amino acid for incorporation into a peptide by a nonribosomal process.